{
  "gene_symbol": "SLC38A7",
  "term_label": "L-glutamine transmembrane transporter activity",
  "term_id": "GO:0015186",
  "gene": "UniProtKB:Q9NVC3",
  "gene_name": "Sodium-coupled neutral amino acid transporter 7"
}